mast cell differentiation [GO:0060374] (biological process) Relationships: is a type of myeloid leukocyte differentiation [GO:0002573] Definition: The process in which a relatively unspecialized myeloid precursor cell acquires the specialized features of a mast cell. A mast cell is a cell that is found in almost all tissues containing numerous basophilic granules and capable of releasing large amounts of histamine and heparin upon activation. Sources: GOC:dph, GOC:tb Regulation: regulated by regulation of mast cell differentiation [GO:0060375]; positively regulated by GO:0060376; RO_0002212 by negative regulation of mast cell differentiation [GO:0060377]